bacterial-type flagellum basal body, distal rod [GO:0009426] (cellular component) Also known as: flagellar basal body, distal rod, flagellin-based flagellum basal body, distal rod References: PMID:10572114, PMID:11133968, PMID:12624192 Sources: GOC:cilia, GOC:mtg_sensu Definition: The portion of the central rod of the bacterial-type flagellar basal body that is distal to the cell membrane; spans most of the distance between the inner and outer membranes. Relationships: is a type of cellular anatomical structure [GO:0110165]; is part of bacterial-type flagellum basal body, rod [GO:0030694]